{
  "term_label": "Unknown cellular component",
  "gene": "UniProtKB:Q6ZVL6",
  "gene_symbol": "KIAA1549L",
  "gene_name": "UPF0606 protein KIAA1549L",
  "term_id": "UNKNOWN:0003"
}